{
  "gene": "UniProtKB:Q8N4T8",
  "gene_name": "3-oxoacyl-[acyl-carrier-protein] reductase",
  "term_label": "Unknown cellular component",
  "gene_symbol": "CBR4",
  "term_id": "UNKNOWN:0003"
}